positive regulation of SNARE complex assembly [GO:0035543] (biological process) Relationships: is_a GO:0031334; is_a positive regulation of vesicle fusion [GO:0031340]; is a type of regulation of SNARE complex assembly [GO:0035542]; positively regulates SNARE complex assembly [GO:0035493] Definition: Any process that increases the frequency, rate or extent of assembly of the SNARE complex. The SNARE complex is a protein complex involved in membrane fusion; a stable ternary complex consisting of a four-helix bundle, usually formed from one R-SNARE and three Q-SNAREs with an ionic layer sandwiched between hydrophobic layers. Sources: GOC:rb